{
  "gene": "UniProtKB:O14647",
  "term_id": "GO:0000785",
  "gene_name": "Chromodomain-helicase-DNA-binding protein 2",
  "gene_symbol": "CHD2",
  "term_label": "chromatin"
}